{
  "term_label": "nucleus",
  "term_id": "GO:0005634",
  "gene": "UniProtKB:Q13151",
  "gene_symbol": "HNRNPA0",
  "gene_name": "Heterogeneous nuclear ribonucleoprotein A0"
}